collagen type VIII trimer [GO:0005591] (cellular component) Definition: A collagen heterotrimer containing type VIII alpha chains; [alpha1(VIII)2]alpha2(VIII) and alpha1(VIII)[alpha2(VIII)]2 trimers have been observed; type VIII collagen triple helices associate to form regular hexagonal nets. References: PMID:21421911 Relationships: is a type of network-forming collagen trimer [GO:0098642]; is part of interstitial hexagonal collagen network [GO:0098646]; is part of hexagonal collagen network of basement membrane [GO:0140155]